{
  "term_label": "phototransduction",
  "term_id": "GO:0007602",
  "gene_name": "Opsin-3",
  "gene": "UniProtKB:Q9H1Y3",
  "gene_symbol": "OPN3"
}